{
  "term_id": "GO:0005813",
  "gene_symbol": "ZFYVE26",
  "gene_name": "Zinc finger FYVE domain-containing protein 26",
  "term_label": "centrosome",
  "gene": "UniProtKB:Q68DK2"
}